asymmetric stem cell division [GO:0098722] (biological process) Subtypes: skeletal muscle satellite stem cell asymmetric division [GO:0014833], germline stem cell asymmetric division [GO:0098728] Relationships: is a type of GO:0008356; is a type of stem cell division [GO:0017145] Definition: Division of a stem cell during which it retains its identity and buds off a daughter cell with a new identity. References: PMID:18513950 Sources: GOC:dos